{
  "gene_name": "Sodium_potassium-transporting ATPase subunit beta-2",
  "gene_symbol": "ATP1B2",
  "gene": "UniProtKB:P14415",
  "term_id": "GO:1990573",
  "term_label": "potassium ion import across plasma membrane"
}